establishment of cell polarity involved in ameboidal cell migration [GO:0003365] (biological process) Definition: The specification and formation of anisotropic intracellular organization that contributes to the self-propelled directed movement of an ameboid cell. Relationships: is a type of GO:0030010; is part of GO:0001667 Sources: GOC:ascb_2009, GOC:dph, GOC:tb Subtypes: establishment of cell polarity involved in gastrulation cell migration [GO:0003379]